ferredoxin-[NAD(P)H] reductase activity [GO:0008937] (molecular function) Relationships: is a type of oxidoreductase activity, acting on iron-sulfur proteins as donors, NAD or NADP as acceptor [GO:0016731] Also known as: ferredoxin reductase activity Subtypes: GO:0004324, ferredoxin-NAD+ reductase activity [GO:0008860] Sources: GOC:curators Definition: Catalysis of the reaction: reduced ferredoxin + NAD(P)+ = oxidized ferredoxin + NAD(P)H + H+.